{
  "term_label": "RNA polymerase II cis-regulatory region sequence-specific DNA binding",
  "gene_symbol": "ZNF876P",
  "term_id": "GO:0000978",
  "gene": "UniProtKB:Q49A33",
  "gene_name": "Putative zinc finger protein 876"
}